{
  "term_id": "GO:0015760",
  "gene": "UniProtKB:Q8TED4",
  "gene_name": "Glucose-6-phosphate exchanger SLC37A2",
  "term_label": "glucose-6-phosphate transport",
  "gene_symbol": "SLC37A2"
}